negative regulation of arbuscule formation for nutrient acquisition from host [GO:0075331] (biological process) Definition: Any process that stops, prevents, or reduces the frequency, rate or extent of symbiont arbuscule formation for nutrient acquisition from host. The host is defined as the larger of the organisms involved in a symbiotic interaction. Relationships: is a type of GO:0044147; is a type of regulation of arbuscule formation for nutrient acquisition from host [GO:0075329]; negatively regulates formation of arbuscule for nutrient acquisition [GO:0075328] Note: Note that this term should not be used to annotate gene products of the host. It should only be used to annotate those gene products from the symbiont involved in this process. Sources: GOC:pamgo_curators